hydroxymethylfurfural reductase (NADPH) activity [GO:0033845] (molecular function) Relationships: is_a GO:0016616 Definition: Catalysis of the reaction: 5-hydroxymethylfurfural + NADPH + H+ = 2,5-bis-hydroxymethylfuran + NADP+. References: PMID:15338422, PMID:16652391 Sources: GOC:jp, GOC:mah